{
  "gene_symbol": "DAPK3",
  "term_id": "GO:0035556",
  "gene": "UniProtKB:O43293",
  "term_label": "intracellular signal transduction",
  "gene_name": "Death-associated protein kinase 3"
}